{
  "gene": "UniProtKB:O60281",
  "term_id": "GO:0000981",
  "term_label": "DNA-binding transcription factor activity, RNA polymerase II-specific",
  "gene_symbol": "ZNF292",
  "gene_name": "Zinc finger protein 292"
}